negative regulation of secretion by cell [GO:1903531] (biological process) Relationships: is a type of negative regulation of cellular process [GO:0048523]; is a type of negative regulation of secretion [GO:0051048]; is a type of regulation of secretion by cell [GO:1903530]; negatively regulates GO:0032940 Subtypes: negative regulation of extracellular matrix constituent secretion [GO:0003332], negative regulation of glutamate secretion [GO:0014050], negative regulation of serotonin secretion [GO:0014063], GO:0032307, negative regulation of catecholamine secretion [GO:0033604], negative regulation of exocytosis [GO:0045920], negative regulation of hormone secretion [GO:0046888], negative regulation of neurotransmitter secretion [GO:0046929], negative regulation of protein secretion [GO:0050709], negative regulation of aspartate secretion [GO:1904449] References: PMID:12130530 Sources: GOC:TermGenie, GOC:pm, GO_REF:0000058 Definition: Any process that stops, prevents or reduces the frequency, rate or extent of secretion by cell. Also known as: down regulation of cellular secretion, down regulation of secretion by cell, down-regulation of cellular secretion, down-regulation of secretion by cell, downregulation of cellular secretion, downregulation of secretion by cell, negative regulation of cellular secretion, inhibition of cellular secretion, inhibition of secretion by cell